{
  "term_id": "GO:0000381",
  "gene_symbol": "SRSF8",
  "gene": "UniProtKB:Q9BRL6",
  "term_label": "regulation of alternative mRNA splicing, via spliceosome",
  "gene_name": "Serine_arginine-rich splicing factor 8"
}